bI3 intron splicing complex [GO:0106392] (cellular component) Relationships: is a type of endoribonuclease complex [GO:1902555] Definition: Aprotein complex required for the splicing of intron 3 of the cytochrome b (COB) gene. In S. cerevisiae, the complex contains the maturase bI3 (which derives from one of the products of the splicing), the MRS1 cofactor and the intron 4 of the cytochrome b pre-mRNA. The two proteins stimulate the ribozyme activity of the pre-mRNA which autoctalyse a group I intron splicing. References: PMID:11773622 Sources: GOC:lnp